calcium,diacylglycerol-dependent serine/threonine kinase activity [GO:0004698] (molecular function) Relationships: is a type of diacylglycerol-dependent serine/threonine kinase activity [GO:0004697]; is_a GO:0009931 References: PMID:34834162 Definition: Calcium-dependent catalysis of the reaction: ATP + a protein = ADP + a phosphoprotein. This reaction is activated in the presence of diacylglycerol and calcium. Also known as: calcium-dependent PKC activity, conventional protein kinase C activity